{
  "term_label": "transcription coregulator activity",
  "gene": "UniProtKB:Q9Y6X2",
  "gene_symbol": "PIAS3",
  "term_id": "GO:0003712",
  "gene_name": "E3 SUMO-protein ligase PIAS3"
}